{
  "gene_name": "Glutamate--cysteine ligase regulatory subunit",
  "term_label": "glutathione biosynthetic process",
  "gene": "UniProtKB:P48507",
  "term_id": "GO:0006750",
  "gene_symbol": "GCLM"
}